{
  "gene_name": "Zinc finger protein 385D",
  "gene": "UniProtKB:Q9H6B1",
  "gene_symbol": "ZNF385D",
  "term_label": "Unknown molecular function",
  "term_id": "UNKNOWN:0001"
}